{
  "term_label": "plasma membrane",
  "gene_name": "Olfactory receptor 10J5",
  "gene": "UniProtKB:Q8NHC4",
  "gene_symbol": "OR10J5",
  "term_id": "GO:0005886"
}